postsynaptic endocytic zone membrane [GO:0098844] (cellular component) Definition: The region of the postsynaptic membrane that is part of the postsynaptic endocytic zone. This region of membrane is associated with stable clathrin puncta. References: PMID:17880892 Relationships: is a type of synaptic membrane [GO:0097060]; is part of postsynaptic membrane [GO:0045211]; is part of postsynaptic endocytic zone [GO:0098843]